{
  "gene": "UniProtKB:Q14692",
  "term_id": "GO:0000462",
  "gene_symbol": "BMS1",
  "term_label": "maturation of SSU-rRNA from tricistronic rRNA transcript (SSU-rRNA, 5.8S rRNA, LSU-rRNA)",
  "gene_name": "Ribosome biogenesis protein BMS1 homolog"
}